{
  "gene": "UniProtKB:Q8NI28",
  "gene_symbol": "RNF32-DT",
  "term_label": "Unknown biological process",
  "term_id": "UNKNOWN:0002",
  "gene_name": "Putative transmenbrane protein RNF32-DT"
}